N-acetyl-beta-glucosaminyl-derivative 4-beta-N-acetylgalactosaminyltransferase activity [GO:0033842] (molecular function) Sources: RHEA:20493 Relationships: is a type of acetylgalactosaminyltransferase activity [GO:0008376] Also known as: N-acetyl-beta-glucosaminyl-glycoprotein 4-beta-N-acetylgalactosaminyltransferase activity, UDP-N-acetyl-D-galactosamine:N-acetyl-D-glucosaminyl-group beta-1,4-N-acetylgalactosaminyltransferase activity, beta1,4-N-acetylgalactosaminyltransferase III activity, beta1,4-N-acetylgalactosaminyltransferase IV activity, beta1,4-N-acetylgalactosaminyltransferase activity, beta4GalNAc-T3, beta4GalNAc-T4 Definition: Catalysis of the reaction: an N-acetyl-beta-D-glucosaminyl derivative + UDP-N-acetyl-alpha-D-galactosamine = an N-acetyl-beta-D-galactosaminyl-(1->4)-N-acetyl-beta-D-glucosaminyl derivative + UDP + H+.